{
  "term_label": "cytoplasm",
  "gene_name": "Kynurenine--oxoglutarate transaminase 3",
  "term_id": "GO:0005737",
  "gene": "UniProtKB:Q6YP21",
  "gene_symbol": "KYAT3"
}